{
  "gene_symbol": "DCDC2C",
  "gene_name": "Doublecortin domain-containing protein 2C",
  "term_label": "microtubule",
  "gene": "UniProtKB:A8MYV0",
  "term_id": "GO:0005874"
}